{
  "gene": "UniProtKB:Q9Y2U5",
  "term_label": "cytosol",
  "gene_name": "Mitogen-activated protein kinase kinase kinase 2",
  "term_id": "GO:0005829",
  "gene_symbol": "MAP3K2"
}